charged-tRNA amino acid modification [GO:0019988] (BP) Relationships: is a type of GO:0006400 Subtypes: GO:0001717, conversion of lysyl-tRNA to pyrrolysyl-tRNA [GO:0001720], GO:0043685, conversion of aspartyl-tRNA to asparaginyl-tRNA [GO:0043688], conversion of methionyl-tRNA to N-formyl-methionyl-tRNA [GO:0071951], GO:0071952 Sources: GOC:jsg Also known as: charged tRNA amino acid modification, charged tRNA modification, pre-translational amino acid modification, pre-translational protein modification, pretranslation protein modification, pretranslational amino acid modification, charged-tRNA modification Definition: The covalent alteration of an amino acid charged on a tRNA before it is incorporated into a protein, as in N-formylmethionine, selenocysteine or pyrrolysine.